{
  "term_label": "Unknown biological process",
  "gene_name": "Uncharacterized protein",
  "term_id": "UNKNOWN:0002",
  "gene_symbol": "A0A804HIB5",
  "gene": "UniProtKB:A0A804HIB5"
}